{
  "term_label": "regulation of protein localization to membrane",
  "term_id": "GO:1905475",
  "gene_name": "Glypican-3",
  "gene_symbol": "GPC3",
  "gene": "UniProtKB:P51654"
}